{
  "gene_symbol": "OR6P1",
  "term_id": "GO:0050911",
  "term_label": "detection of chemical stimulus involved in sensory perception of smell",
  "gene": "UniProtKB:Q8NGX9",
  "gene_name": "Olfactory receptor 6P1"
}